{
  "term_id": "GO:0030667",
  "gene": "UniProtKB:P09172",
  "gene_symbol": "DBH",
  "term_label": "secretory granule membrane",
  "gene_name": "Dopamine beta-hydroxylase"
}